response to hydrogen sulfide [GO:1904880] (biological process) Definition: Any process that results in a change in state or activity of a cell or an organism (in terms of movement, secretion, enzyme production, gene expression, etc.) as a result of a hydrogen sulfide stimulus. References: PMID:24012591 Sources: GOC:TermGenie, GO_REF:0000071 Also known as: response to dihydridosulfur, response to sulfane Relationships: is a type of response to chemical [GO:0042221] Subtypes: cellular response to hydrogen sulfide [GO:1904881]